regulation of conidiophore development [GO:0070793] (biological process) Relationships: is a type of GO:0075260; regulates GO:0070787 Definition: Any process that modulates the frequency, rate or extent of conidiophore development, a process that leads to the formation of a conidiophore. The conidiophore is a specialized hypha that extends aerially from the growth substrate and bears conidia, or asexual spores. Subtypes: GO:0070794, positive regulation of conidiophore development [GO:0070795], GO:0070802 Sources: GOC:mah